{
  "gene_symbol": "ACSS2",
  "term_label": "acetate-CoA ligase activity",
  "gene_name": "Acetyl-coenzyme A synthetase, cytoplasmic",
  "term_id": "GO:0003987",
  "gene": "UniProtKB:Q9NR19"
}